{
  "gene": "UniProtKB:P0DPK5",
  "gene_symbol": "H3Y2",
  "term_id": "GO:0030527",
  "term_label": "structural constituent of chromatin",
  "gene_name": "Histone H3.X"
}